{
  "gene_symbol": "DGKH",
  "gene_name": "Diacylglycerol kinase eta",
  "term_id": "GO:0006654",
  "term_label": "phosphatidic acid biosynthetic process",
  "gene": "UniProtKB:Q86XP1"
}